{
  "gene_symbol": "SAP30L",
  "gene": "UniProtKB:Q9HAJ7",
  "gene_name": "Histone deacetylase complex subunit SAP30L",
  "term_label": "histone deacetylase complex",
  "term_id": "GO:0000118"
}